{
  "gene": "UniProtKB:Q9H0A6",
  "gene_symbol": "RNF32",
  "gene_name": "RING finger protein 32",
  "term_id": "UNKNOWN:0002",
  "term_label": "Unknown biological process"
}